{
  "term_label": "DNA-binding transcription factor activity, RNA polymerase II-specific",
  "term_id": "GO:0000981",
  "gene": "UniProtKB:Q9UJN7",
  "gene_name": "Zinc finger protein 391",
  "gene_symbol": "ZNF391"
}